{
  "gene_name": "Cyclic AMP-responsive element-binding protein 3",
  "term_label": "RNA polymerase II cis-regulatory region sequence-specific DNA binding",
  "gene_symbol": "CREB3",
  "term_id": "GO:0000978",
  "gene": "UniProtKB:O43889"
}